{
  "gene_name": "FAST kinase domain-containing protein 1, mitochondrial",
  "gene": "UniProtKB:Q53R41",
  "term_label": "ribonucleoprotein granule",
  "gene_symbol": "FASTKD1",
  "term_id": "GO:0035770"
}